{
  "gene": "UniProtKB:Q9HBW1",
  "gene_symbol": "LRRC4",
  "gene_name": "Leucine-rich repeat-containing protein 4",
  "term_label": "excitatory synapse assembly",
  "term_id": "GO:1904861"
}